{
  "term_label": "tumor necrosis factor receptor activity",
  "term_id": "GO:0005031",
  "gene_symbol": "TNFRSF11A",
  "gene_name": "Tumor necrosis factor receptor superfamily member 11A",
  "gene": "UniProtKB:Q9Y6Q6"
}